D-cysteine desulfhydrase activity [GO:0019148] (molecular function) Relationships: is a type of carbon-sulfur lyase activity [GO:0016846] Also known as: D-cysteine lyase activity, D-cysteine sulfide-lyase (deaminating), D-cysteine sulfide-lyase (deaminating; pyruvate-forming) Sources: EC:4.4.1.15 Definition: Catalysis of the reaction: D-cysteine + H2O = sulfide + NH3 + pyruvate.